{
  "term_label": "kinase activity",
  "gene": "UniProtKB:Q8IV42",
  "term_id": "GO:0016301",
  "gene_name": "L-seryl-tRNA(Sec) kinase",
  "gene_symbol": "PSTK"
}